cerebellar granule cell precursor tangential migration [GO:0021935] (BP) References: PMID:15157725 Sources: GOC:cls, GOC:dgh, GOC:dph, GOC:jid, GO_REF:0000021 Definition: The early migration of granule cell precursors in which cells move orthogonal to the direction of radial migration and ultimately cover the superficial zone of the cerebellar primordium. Relationships: is a type of hindbrain tangential cell migration [GO:0021934]